{
  "term_label": "Unknown cellular component",
  "term_id": "UNKNOWN:0003",
  "gene_name": "Leucine-rich repeat flightless-interacting protein 2",
  "gene": "UniProtKB:Q9Y608",
  "gene_symbol": "LRRFIP2"
}